{
  "term_label": "Unknown biological process",
  "gene_name": "Carbonic anhydrase 1",
  "term_id": "UNKNOWN:0002",
  "gene_symbol": "CA1",
  "gene": "UniProtKB:P00915"
}